silver ion transmembrane transporter activity [GO:0015080] (MF) Relationships: is a type of GO:0046915; is part of silver ion transmembrane transport [GO:1902601] Sources: GOC:ai Subtypes: P-type silver transporter activity [GO:0015445] Definition: Enables the transfer of silver (Ag+) ions from one side of a membrane to the other. Also known as: silver transporter activity